{
  "gene": "UniProtKB:Q7RTP6",
  "gene_name": "[F-actin]-monooxygenase MICAL3",
  "term_label": "oxidoreductase activity, acting on paired donors, with incorporation or reduction of molecular oxygen, NAD(P)H as one donor, and incorporation of one atom of oxygen",
  "gene_symbol": "MICAL3",
  "term_id": "GO:0016709"
}